{
  "term_id": "GO:0005634",
  "term_label": "nucleus",
  "gene_symbol": "CALML3",
  "gene": "UniProtKB:P27482",
  "gene_name": "Calmodulin-like protein 3"
}